{
  "term_label": "Unknown cellular component",
  "gene_symbol": "PEF1",
  "gene": "UniProtKB:Q9UBV8",
  "term_id": "UNKNOWN:0003",
  "gene_name": "Peflin"
}